{
  "term_id": "GO:0005829",
  "gene_name": "Carbonic anhydrase 3",
  "term_label": "cytosol",
  "gene": "UniProtKB:P07451",
  "gene_symbol": "CA3"
}